{
  "gene_symbol": "TFAP2D",
  "gene_name": "Transcription factor AP-2-delta",
  "term_label": "nucleus",
  "gene": "UniProtKB:Q7Z6R9",
  "term_id": "GO:0005634"
}